myristoyl-CoA ligase activity [GO:0090432] (molecular function) References: PMID:18071249 Sources: GOC:al Also known as: myristoyl-CoA synthetase activity Relationships: is a type of long-chain fatty acid-CoA ligase activity [GO:0004467] Definition: Catalysis of the reaction: ATP + myristic acid + CoA = AMP + diphosphate + myristoyl-CoA.